secologanin synthase activity [GO:0050616] (molecular function) Sources: EC:1.14.19.62, MetaCyc:1.3.3.9-RXN Also known as: loganin:oxygen oxidoreductase (ring-cleaving) Relationships: is_a oxidoreductase activity, acting on the CH-CH group of donors, oxygen as acceptor [GO:0016634] Definition: Catalysis of the reaction: loganin + NADPH + H+ + O2 = secologanin + NADP+ + 2 H2O.